{
  "gene_symbol": "FAM161B",
  "term_label": "Unknown molecular function",
  "term_id": "UNKNOWN:0001",
  "gene_name": "Protein FAM161B",
  "gene": "UniProtKB:Q96MY7"
}